positive regulation of glycoprotein biosynthetic process involved in immunological synapse formation [GO:2000526] (biological process) Relationships: is a type of GO:0010560; is part of immunological synapse formation [GO:0001771] Definition: Any positive regulation of glycoprotein biosynthetic process that is involved in immunological synapse formation. Sources: GOC:obol Also known as: positive regulation of glycoprotein biosynthetic process of formation of immunological synapse, positive regulation of glycoprotein biosynthetic process of immunological synapse formation